paclitaxel biosynthetic process [GO:0042617] (biological process) Sources: GOC:jl, GOC:krc Relationships: is_a diterpenoid biosynthetic process [GO:0016102] Definition: The chemical reactions and pathways resulting in the formation of paclitaxel, a tetracyclic diterpenoid isolated originally from the bark of the Pacific yew tree, Taxus brevifolia. Also known as: paclitaxel metabolic process, paclitaxel metabolism, taxol metabolic process, taxol metabolism, paclitaxel anabolism, paclitaxel biosynthesis, paclitaxel formation, paclitaxel synthesis, taxol biosynthesis, taxol biosynthetic process